{
  "gene_symbol": "TLN2",
  "term_id": "GO:0005925",
  "gene_name": "Talin-2",
  "gene": "UniProtKB:Q9Y4G6",
  "term_label": "focal adhesion"
}